regulation of organohalogen metabolic process [GO:0090347] (biological process) Definition: Any process that modulates the rate, frequency or extent of the chemical reactions and pathways involving organohalogen compounds, as carried out by individual cells. Sources: GOC:BHF Relationships: is a type of regulation of metabolic process [GO:0019222]; regulates organohalogen metabolic process [GO:0090345] Subtypes: negative regulation of organofluorine metabolic process [GO:0090350]